{
  "gene_name": "Charged multivesicular body protein 2b",
  "gene_symbol": "CHMP2B",
  "term_id": "GO:0032509",
  "term_label": "endosome transport via multivesicular body sorting pathway",
  "gene": "UniProtKB:Q9UQN3"
}